microtubule nucleation by spindle pole body [GO:0051417] (biological process) Definition: The 'de novo' formation of a microtubule, mediated by the spindle pole body. Sources: GOC:ai Relationships: is a type of microtubule nucleation by microtubule organizing center [GO:0051418] Also known as: SPB-mediated microtubule nucleation, microtubule nucleation by SPB, spindle pole body-mediated microtubule nucleation